{
  "gene": "UniProtKB:P80162",
  "term_label": "antimicrobial humoral immune response mediated by antimicrobial peptide",
  "gene_symbol": "CXCL6",
  "term_id": "GO:0061844",
  "gene_name": "C-X-C motif chemokine 6"
}